chloroplast thylakoid membrane protein complex [GO:0098807] (cellular component) Sources: GOC:dos Definition: A protein complex that is part of a chloroplast thylakoid membrane. Relationships: is a type of membrane protein complex [GO:0098796]; is part of chloroplast thylakoid membrane [GO:0009535] Subtypes: GO:0009503, GO:0009655, PSII associated light-harvesting complex II, peripheral complex [GO:0009656], GO:0030085, chloroplast photosystem I [GO:0030093], chloroplast photosystem II [GO:0030095]